{
  "gene_symbol": "OR2B11",
  "gene_name": "Olfactory receptor 2B11",
  "gene": "UniProtKB:Q5JQS5",
  "term_label": "plasma membrane",
  "term_id": "GO:0005886"
}